{
  "gene_name": "Zinc finger BED domain-containing protein 5",
  "term_label": "Unknown molecular function",
  "gene_symbol": "ZBED5",
  "term_id": "UNKNOWN:0001",
  "gene": "UniProtKB:Q49AG3"
}